peptidyl-histidine adenylylation [GO:0051111] (biological process) Definition: The adenylylation of peptidyl-histidine to form peptidyl-1'-(phospho-5'-adenosine)-L-histidine (otherwise known as tau-AMP-histidine, tele-AMP-histidine) or peptidyl-3'-(phospho-5'-adenosine)-L-histidine (otherwise known as pi-AMP-histidine, pros-AMP-histidine). Sources: RESID:AA0371 Relationships: is a type of GO:0018117; is_a peptidyl-histidine modification [GO:0018202]